{
  "gene": "UniProtKB:Q03164",
  "term_id": "GO:0035097",
  "gene_symbol": "KMT2A",
  "gene_name": "Histone-lysine N-methyltransferase 2A",
  "term_label": "histone methyltransferase complex"
}